{
  "gene_symbol": "SAR1A",
  "gene_name": "GTP-binding protein SAR1a",
  "gene": "UniProtKB:Q9NR31",
  "term_label": "vesicle organization",
  "term_id": "GO:0016050"
}